membrane repolarization during bundle of His cell action potential [GO:0086050] (biological process) Definition: The process in which ions are transported across a membrane such that the bundle of His cardiac muscle cell membrane potential changes in the direction from the positive membrane potential at the peak of the action potential towards the negative resting potential. Also known as: membrane repolarization during bundle of His cardiac muscle cell action potential Relationships: is a type of membrane repolarization during cardiac muscle cell action potential [GO:0086013]; is part of bundle of His cell action potential [GO:0086043] Sources: GOC:BHF, GOC:dph, GOC:mtg_cardiac_conduct_nov11